{
  "gene": "UniProtKB:P07359",
  "gene_name": "Platelet glycoprotein Ib alpha chain",
  "term_label": "blood coagulation, intrinsic pathway",
  "term_id": "GO:0007597",
  "gene_symbol": "GP1BA"
}